GDP-L-galactose phosphorylase activity [GO:0080047] (MF) Relationships: is a type of GO:0070568 References: PMID:17462988, PMID:18463094 Sources: RHEA:27698 Also known as: GDP:galactose-1-phosphate guanyltransferase activity, galactose-1-phosphate guanylyltransferase (GDP) activity Definition: Catalysis of the reaction: GDP-beta-L-galactose + phosphate = beta-L-galactose-1-phosphate + GDP.